{
  "gene_symbol": "SYNM",
  "gene_name": "Synemin",
  "term_label": "structural constituent of cytoskeleton",
  "term_id": "GO:0005200",
  "gene": "UniProtKB:O15061"
}